{
  "term_label": "Unknown biological process",
  "gene_name": "Golgi-associated RAB2 interactor protein 1B",
  "gene_symbol": "GARIN1B",
  "term_id": "UNKNOWN:0002",
  "gene": "UniProtKB:Q96KD3"
}